3',5'-cyclic-GMP phosphodiesterase activity [GO:0047555] (molecular function) Sources: RHEA:16957 Also known as: 3',5' cyclic-GMP phosphodiesterase activity, cGMP phosphodiesterase activity, cGMP-specific phosphodiesterase activity, cyclic GMP phosphodiesterase activity, guanosine cyclic 3',5'-phosphate phosphodiesterase activity, 3',5'-cyclic-GMP 5'-nucleotidohydrolase activity, cGMP-PDE, cyclic 3',5'-GMP phosphodiesterase activity, cyclic guanosine 3',5'-monophosphate phosphodiesterase activity, cyclic guanosine 3',5'-phosphate phosphodiesterase activity Subtypes: GO:0004117, calmodulin-activated 3',5'-cyclic-GMP phosphodiesterase activity [GO:0048101] Definition: Catalysis of the reaction: 3',5'-cyclic GMP + H2O = GMP + H+. Relationships: is a type of 3',5'-cyclic-nucleotide phosphodiesterase activity [GO:0004114]